{
  "gene_name": "Protein cornichon homolog 4",
  "term_id": "GO:0005789",
  "term_label": "endoplasmic reticulum membrane",
  "gene": "UniProtKB:Q9P003",
  "gene_symbol": "CNIH4"
}